citrate-CoA ligase activity [GO:0047779] (molecular function) Also known as: citrate thiokinase activity, citrate:CoA ligase (ADP-forming), citrate:CoA ligase activity, citryl-CoA synthetase activity Sources: EC:6.2.1.18, RHEA:21472 Definition: Catalysis of the reaction: ATP + citrate + CoA = (3S)-citryl-CoA + ADP + H+ + phosphate. Relationships: is a type of acid-thiol ligase activity [GO:0016878]